{
  "gene_name": "40-kDa huntingtin-associated protein",
  "term_label": "vesicle cytoskeletal trafficking",
  "gene": "UniProtKB:P23610",
  "gene_symbol": "F8A3",
  "term_id": "GO:0099518"
}